{
  "gene_name": "Vesicle transport through interaction with t-SNAREs homolog 1B",
  "term_id": "GO:0031201",
  "gene": "UniProtKB:Q9UEU0",
  "term_label": "SNARE complex",
  "gene_symbol": "VTI1B"
}